{
  "gene": "UniProtKB:Q9NRZ9",
  "gene_symbol": "HELLS",
  "gene_name": "Lymphoid-specific helicase",
  "term_id": "GO:0031508",
  "term_label": "pericentric heterochromatin formation"
}